{
  "gene_symbol": "ANXA10",
  "gene_name": "Annexin A10",
  "term_id": "UNKNOWN:0002",
  "term_label": "Unknown biological process",
  "gene": "UniProtKB:Q9UJ72"
}